{
  "gene_name": "Cysteine-rich protein 1",
  "term_id": "GO:0008270",
  "term_label": "zinc ion binding",
  "gene": "UniProtKB:P50238",
  "gene_symbol": "CRIP1"
}